peroxisomal membrane transport [GO:0015919] (biological process) Subtypes: long-chain fatty acid import into peroxisome [GO:0015910], GO:0016558, GO:0045046 Definition: The directed movement of substances to, from or across the peroxisomal membrane. Relationships: is a type of GO:0043574 Sources: GOC:ai